{
  "gene_name": "Serine_threonine-protein phosphatase 2A 55 kDa regulatory subunit B gamma isoform",
  "gene_symbol": "PPP2R2C",
  "gene": "UniProtKB:Q9Y2T4",
  "term_id": "UNKNOWN:0002",
  "term_label": "Unknown biological process"
}